type I pneumocyte differentiation [GO:0060509] (biological process) Relationships: is a type of lung epithelial cell differentiation [GO:0060487] Definition: The process in which a relatively unspecialized cell acquires specialized features of a type I pneumocyte. A type I pneumocyte is a flattened cell with greatly attenuated cytoplasm and a paucity of organelles. Sources: GOC:dph, GOC:mtg_lung, ISBN:0721662544 Also known as: membranous pneumocyte differentiation, small alveolar cell differentiation, squamous alveolar cell differentiation